{
  "gene_symbol": "PSAP",
  "term_label": "regulation of lipid metabolic process",
  "gene": "UniProtKB:P07602",
  "gene_name": "Prosaposin",
  "term_id": "GO:0019216"
}